{
  "term_label": "Unknown cellular component",
  "gene": "UniProtKB:Q8TCU3",
  "gene_name": "Solute carrier family 7 member 13",
  "term_id": "UNKNOWN:0003",
  "gene_symbol": "SLC7A13"
}